multiplexin collagen trimer [GO:0140156] (cellular component) Subtypes: GO:0005582, GO:0030938 References: PMID:21421911, PMID:27746220, PMID:31479735, PMID:33543021 Definition: Collagen that contains multiple triple-helix domains with interruptions. Relationships: is a type of collagen trimer [GO:0005581]; is part of collagenous component of basement membrane [GO:0140143]